{
  "gene_name": "Sulfotransferase 1A4",
  "term_label": "cytoplasm",
  "gene": "UniProtKB:P0DMN0",
  "term_id": "GO:0005737",
  "gene_symbol": "SULT1A4"
}